{
  "gene_name": "Probable oxidoreductase PXDNL",
  "gene_symbol": "PXDNL",
  "term_id": "GO:0004601",
  "term_label": "peroxidase activity",
  "gene": "UniProtKB:A1KZ92"
}